{
  "gene_symbol": "UNQ9165_PRO28630",
  "gene_name": "Putative uncharacterized protein UNQ9165_PRO28630",
  "term_label": "Unknown cellular component",
  "term_id": "UNKNOWN:0003",
  "gene": "UniProtKB:Q6UXU0"
}